{
  "term_id": "GO:0045893",
  "gene_symbol": "ANKRD49",
  "gene_name": "Ankyrin repeat domain-containing protein 49",
  "term_label": "positive regulation of DNA-templated transcription",
  "gene": "UniProtKB:Q8WVL7"
}